{
  "gene_symbol": "A0A7I2V2S6",
  "gene_name": "Uncharacterized protein",
  "gene": "UniProtKB:A0A7I2V2S6",
  "term_id": "UNKNOWN:0003",
  "term_label": "Unknown cellular component"
}